regulation of thrombin-activated receptor signaling pathway [GO:0070494] (biological process) Definition: Any process that modulates the frequency, rate or extent of a thrombin-activated receptor signaling pathway activity. A thrombin receptor signaling pathway is the series of molecular signals generated as a consequence of a thrombin-activated receptor binding to one of its physiological ligands. Relationships: is_a regulation of G protein-coupled receptor signaling pathway [GO:0008277]; regulates thrombin-activated receptor signaling pathway [GO:0070493] Also known as: regulation of thrombin receptor signaling pathway, regulation of thrombin receptor signalling pathway Sources: GOC:mah Subtypes: GO:0070495, positive regulation of thrombin-activated receptor signaling pathway [GO:0070496]